{
  "term_label": "plasma membrane",
  "gene_name": "Transient receptor potential cation channel subfamily V member 1",
  "gene": "UniProtKB:Q8NER1",
  "term_id": "GO:0005886",
  "gene_symbol": "TRPV1"
}